{
  "gene_symbol": "PDE2A",
  "term_label": "3',5'-cGMP-stimulated cyclic-nucleotide phosphodiesterase activity",
  "term_id": "GO:0004118",
  "gene": "UniProtKB:O00408",
  "gene_name": "cGMP-dependent 3',5'-cyclic phosphodiesterase"
}